{
  "term_id": "GO:0005886",
  "term_label": "plasma membrane",
  "gene": "UniProtKB:Q8NGY9",
  "gene_name": "Olfactory receptor 2L8",
  "gene_symbol": "OR2L8"
}